{
  "term_label": "Unknown molecular function",
  "term_id": "UNKNOWN:0001",
  "gene_symbol": "PLBD1",
  "gene_name": "Phospholipase B-like 1",
  "gene": "UniProtKB:Q6P4A8"
}